{
  "gene_name": "Capping protein, Arp2_3 and myosin-I linker protein 3",
  "gene": "UniProtKB:Q8ND23",
  "gene_symbol": "CARMIL3",
  "term_id": "GO:0016477",
  "term_label": "cell migration"
}